{
  "gene_symbol": "VIPR1",
  "term_label": "adenylate cyclase-modulating G protein-coupled receptor signaling pathway",
  "gene": "UniProtKB:P32241",
  "gene_name": "Vasoactive intestinal polypeptide receptor 1",
  "term_id": "GO:0007188"
}